positive regulation of oogonium development [GO:0075265] (BP) Definition: Any process that activates, maintains or increases the frequency, rate or extent of oogonium development, a process that leads to the formation of a female gametangium of oomycetes, containing one or more gametes. Sources: GOC:pamgo_curators Relationships: is a type of positive regulation of spore-bearing organ development [GO:0075261]; is a type of regulation of oogonium development [GO:0075264]; positively regulates oogonium development [GO:0075263]